regulation of cell-cell adhesion involved in gastrulation [GO:0070587] (biological process) References: PMID:19091770 Sources: GOC:dsf Relationships: is a type of regulation of cell-cell adhesion [GO:0022407]; regulates cell-cell adhesion involved in gastrulation [GO:0070586] Definition: Any process that modulates the frequency, rate, or extent of attachment of a cell to another cell affecting gastrulation. Subtypes: negative regulation of heterotypic cell-cell adhesion [GO:0034115]